{
  "term_id": "GO:0007186",
  "gene_symbol": "GPR151",
  "gene_name": "G-protein coupled receptor 151",
  "term_label": "G protein-coupled receptor signaling pathway",
  "gene": "UniProtKB:Q8TDV0"
}